positive regulation of autophagosome-lysosome fusion [GO:0160177] (BP) References: PMID:38360932 Definition: Any process that activates or increases the rate which autophagosomes fuse with a vacuole (yeast) or lysosome (e.g. mammals and insects). Relationships: is a type of positive regulation of vesicle fusion [GO:0031340]; positively regulates autophagosome-lysosome fusion [GO:0061909]